{
  "gene_symbol": "SLC24A3",
  "term_id": "GO:0005886",
  "gene": "UniProtKB:Q9HC58",
  "term_label": "plasma membrane",
  "gene_name": "Sodium_potassium_calcium exchanger 3"
}